{
  "gene_symbol": "MMP24",
  "term_label": "collagen catabolic process",
  "term_id": "GO:0030574",
  "gene": "UniProtKB:Q9Y5R2",
  "gene_name": "Matrix metalloproteinase-24"
}